porphobilinogen synthase activity [GO:0004655] (molecular function) Sources: EC:4.2.1.24, RHEA:24064 Also known as: aminolevulinate dehydratase activity, delta-aminolevulinic acid dehydratase activity, 5-aminolevulinate hydro-lyase (adding 5-aminolevulinate and cyclizing), 5-aminolevulinate hydro-lyase (adding 5-aminolevulinate and cyclizing; porphobilinogen-forming), 5-levulinic acid dehydratase activity, aminolevulinic dehydratase activity, delta-aminolevulinate dehydratase activity, delta-aminolevulinic acid dehydrase activity, delta-aminolevulinic dehydratase activity Relationships: is a type of GO:0016836 Definition: Catalysis of the reaction: 2 5-aminolevulinate = 2 H2O + H+ + porphobilinogen.